{
  "gene": "UniProtKB:Q8IUS5",
  "gene_name": "Epoxide hydrolase 4",
  "term_id": "UNKNOWN:0003",
  "gene_symbol": "EPHX4",
  "term_label": "Unknown cellular component"
}